{
  "term_id": "UNKNOWN:0001",
  "gene": "UniProtKB:P07357",
  "gene_symbol": "C8A",
  "gene_name": "Complement component C8 alpha chain",
  "term_label": "Unknown molecular function"
}